{
  "gene": "UniProtKB:Q14691",
  "gene_name": "DNA replication complex GINS protein PSF1",
  "term_id": "UNKNOWN:0001",
  "term_label": "Unknown molecular function",
  "gene_symbol": "GINS1"
}